{
  "term_id": "GO:0006357",
  "gene": "UniProtKB:P31273",
  "gene_symbol": "HOXC8",
  "gene_name": "Homeobox protein Hox-C8",
  "term_label": "regulation of transcription by RNA polymerase II"
}